{
  "term_label": "Unknown biological process",
  "term_id": "UNKNOWN:0002",
  "gene_name": "TLC domain-containing protein 5",
  "gene_symbol": "TLCD5",
  "gene": "UniProtKB:Q6ZRR5"
}